{
  "gene_name": "Aldo-keto reductase family 1 member B10",
  "gene_symbol": "AKR1B10",
  "gene": "UniProtKB:O60218",
  "term_label": "cytosol",
  "term_id": "GO:0005829"
}